formation of arbuscule for nutrient acquisition [GO:0075328] (biological process) Relationships: is a type of formation of specialized structure for nutrient acquisition [GO:0052093] Sources: GOC:pamgo_curators Regulation: regulated by GO:0075329; positively regulated by positive regulation of arbuscule formation for nutrient acquisition from host [GO:0075330]; negatively regulated by negative regulation of arbuscule formation for nutrient acquisition from host [GO:0075331] Note: Note that this term should not be used to annotate gene products of the host. It should only be used to annotate those gene products from the symbiont involved in this process. Definition: The assembly of an arbuscule, a fine, tree-like hyphal symbiont structure projected into the host cell for the purpose of obtaining nutrients. The host is defined as the larger of the organisms involved in a symbiotic interaction. Also known as: formation by symbiont of arbuscule for nutrient acquisition from host